dishabituation [GO:0097270] (biological process) References: PMID:11390637 Sources: GOC:kmv, Wikipedia:Habituation Definition: The temporary recovery of response to a stimulus when a novel stimulus is added. Relationships: is a type of nonassociative learning [GO:0046958]